{
  "gene_symbol": "RUVBL1",
  "term_label": "R2TP complex",
  "gene": "UniProtKB:Q9Y265",
  "term_id": "GO:0097255",
  "gene_name": "RuvB-like 1"
}